{
  "gene_symbol": "MT1G",
  "gene_name": "Metallothionein-1G",
  "term_label": "cytoplasm",
  "term_id": "GO:0005737",
  "gene": "UniProtKB:P13640"
}